{
  "gene_name": "Dual serine_threonine and tyrosine protein kinase",
  "term_label": "Unknown molecular function",
  "term_id": "UNKNOWN:0001",
  "gene": "UniProtKB:Q6XUX3",
  "gene_symbol": "DSTYK"
}